{
  "gene": "UniProtKB:P15309",
  "term_id": "GO:0016791",
  "gene_symbol": "ACP3",
  "gene_name": "Prostatic acid phosphatase",
  "term_label": "phosphatase activity"
}